electron-transferring-flavoprotein dehydrogenase activity [GO:0004174] (molecular function) Definition: Catalysis of the reaction: a ubiquinone + reduced [electron-transfer flavoprotein] = a ubiquinol + H+ + oxidized [electron-transfer flavoprotein]. Relationships: is a type of GO:0009055; is a type of GO:0016649; is part of respiratory electron transport chain [GO:0022904] Sources: RHEA:24052 Also known as: ETF dehydrogenase activity, ETF-QO activity, ETF-ubiquinone oxidoreductase activity, ETF:ubiquinone oxidoreductase activity, electron transfer flavoprotein Q oxidoreductase activity, electron transfer flavoprotein dehydrogenase activity, electron transfer flavoprotein reductase activity, electron transfer flavoprotein-ubiquinone oxidoreductase activity, electron-transferring-flavoprotein:ubiquinone oxidoreductase activity